protein storage vacuole organization [GO:1990019] (biological process) References: PMID:21670741 Sources: GOC:tb Relationships: is a type of GO:0007033 Definition: A process that is carried out at the cellular level which results in the assembly, arrangement of constituent parts, or disassembly of a protein storage vacuole, a storage vacuole that contains a lytic vacuole.